{
  "gene_name": "Molecular chaperone MKKS",
  "term_label": "developmental process",
  "gene_symbol": "MKKS",
  "term_id": "GO:0032502",
  "gene": "UniProtKB:Q9NPJ1"
}